{
  "gene_name": "Cytochrome P450 4A22",
  "gene": "UniProtKB:Q5TCH4",
  "gene_symbol": "CYP4A22",
  "term_label": "alkane 1-monooxygenase activity",
  "term_id": "GO:0018685"
}